peristromal region viral factory [GO:0039721] (cellular component) Definition: A nuclear viral factory formed at the periphery of the host cell nucleus by Baculoviruses. Also known as: PR References: PMID:18434402 Sources: VZ:1951 Relationships: is a type of GO:0039715